{
  "gene_symbol": "KEAP1",
  "term_label": "proteasome-mediated ubiquitin-dependent protein catabolic process",
  "gene": "UniProtKB:Q14145",
  "gene_name": "Kelch-like ECH-associated protein 1",
  "term_id": "GO:0043161"
}